{
  "gene_symbol": "NSUN2",
  "term_id": "GO:0030488",
  "gene": "UniProtKB:Q08J23",
  "gene_name": "RNA cytosine C(5)-methyltransferase NSUN2",
  "term_label": "tRNA methylation"
}